DNA loop anchor binding [GO:0141094] (molecular function) Definition: Binding to a DNA loop anchor, a region of chromosome that defines the ends of a DNA loop where two parts of same DNA strand are held in close physical proximity. For example, in animals, the anchors of DNA loops are convergently oriented CTCF binding sites during interphase. References: PMID:25497547, PMID:26499245 Relationships: is a type of sequence-specific DNA binding [GO:0043565]